SCF-Pof5 ubiquitin ligase complex [GO:0097672] (cellular component) Relationships: is a type of SCF ubiquitin ligase complex [GO:0019005] Also known as: SCF-YDR306C ubiquitin ligase complex References: PMID:14747994, PMID:15147268 Sources: GOC:jd, GOC:vw Definition: An SCF ubiquitin ligase complex in which the F-box protein is Pof5 in S. pombe (YDR306C in S. cerevisiae).